protein localization to spindle microtubule [GO:1902889] (biological process) References: PMID:16054030 Sources: GOC:TermGenie, GOC:kmv, GO_REF:0000087 Definition: A process in which a protein is transported to, or maintained in, a location within a spindle microtubule. Also known as: protein localisation in spindle microtubule, protein localisation to spindle microtubule, protein localization in spindle microtubule Subtypes: protein localization to polar microtubule [GO:0160086], GO:1902888 Relationships: is a type of protein localization to microtubule [GO:0035372]